{
  "term_label": "nucleotide-excision repair",
  "term_id": "GO:0006289",
  "gene": "UniProtKB:Q8NHY5",
  "gene_name": "Checkpoint protein HUS1B",
  "gene_symbol": "HUS1B"
}